{
  "term_label": "protein import into peroxisome matrix",
  "gene_name": "Peroxisomal ATPase PEX1",
  "term_id": "GO:0016558",
  "gene": "UniProtKB:O43933",
  "gene_symbol": "PEX1"
}